{
  "term_id": "GO:0016020",
  "term_label": "membrane",
  "gene_name": "V-set and transmembrane domain-containing protein 4",
  "gene": "UniProtKB:Q8IW00",
  "gene_symbol": "VSTM4"
}